{
  "gene": "UniProtKB:Q8WTW3",
  "gene_name": "Conserved oligomeric Golgi complex subunit 1",
  "term_id": "UNKNOWN:0001",
  "gene_symbol": "COG1",
  "term_label": "Unknown molecular function"
}